negative regulation of response to oxidative stress [GO:1902883] (biological process) Definition: Any process that stops, prevents or reduces the frequency, rate or extent of response to oxidative stress. Also known as: down regulation of response to oxidative stress, down-regulation of response to oxidative stress, downregulation of response to oxidative stress, inhibition of response to oxidative stress References: PMID:16899554 Sources: GOC:TermGenie, GOC:kmv, GO_REF:0000058 Relationships: is a type of negative regulation of response to stimulus [GO:0048585]; is a type of regulation of response to oxidative stress [GO:1902882]; negatively regulates response to oxidative stress [GO:0006979] Subtypes: negative regulation of cellular response to oxidative stress [GO:1900408], GO:1901032